{
  "term_label": "Unknown molecular function",
  "gene_name": "Voltage-dependent L-type calcium channel subunit beta-2",
  "gene_symbol": "CACNB2",
  "term_id": "UNKNOWN:0001",
  "gene": "UniProtKB:Q08289"
}